{
  "gene": "UniProtKB:P49959",
  "term_label": "double-strand break repair via homologous recombination",
  "gene_name": "Double-strand break repair protein MRE11",
  "term_id": "GO:0000724",
  "gene_symbol": "MRE11"
}